{
  "gene": "UniProtKB:Q8NGN3",
  "term_label": "plasma membrane",
  "term_id": "GO:0005886",
  "gene_symbol": "OR10G4",
  "gene_name": "Olfactory receptor 10G4"
}